regulation of non-canonical Wnt signaling pathway [GO:2000050] (biological process) Also known as: regulation of beta-catenin-independent Wnt receptor signaling pathway, regulation of non-canonical Wnt receptor signaling pathway, regulation of non-canonical Wnt receptor signalling pathway, regulation of non-canonical Wnt-activated signaling pathway Subtypes: GO:0008591, regulation of Frizzled Nuclear Import pathway [GO:0140710], GO:2000051, positive regulation of non-canonical Wnt signaling pathway [GO:2000052], GO:2000095 Sources: GOC:obol, GOC:yaf Definition: Any process that modulates the frequency, rate or extent of non-canonical Wnt signaling pathway. Relationships: is a type of regulation of Wnt signaling pathway [GO:0030111]; regulates non-canonical Wnt signaling pathway [GO:0035567]